regulation of phosphatidylcholine biosynthetic process [GO:2001245] (biological process) Definition: Any process that modulates the frequency, rate or extent of phosphatidylcholine biosynthetic process. Also known as: regulation of phosphatidylcholine anabolism, regulation of phosphatidylcholine biosynthesis, regulation of phosphatidylcholine formation, regulation of phosphatidylcholine synthesis Relationships: is_a GO:0071071; is_a regulation of phosphatidylcholine metabolic process [GO:0150172]; regulates GO:0006656 Subtypes: GO:2001246, GO:2001247 Sources: GOC:obol